{
  "term_id": "GO:0038187",
  "gene": "UniProtKB:Q8WXI8",
  "gene_name": "C-type lectin domain family 4 member D",
  "term_label": "pattern recognition receptor activity",
  "gene_symbol": "CLEC4D"
}